{
  "term_label": "transcription coregulator activity",
  "gene": "UniProtKB:Q9Y2W1",
  "gene_symbol": "THRAP3",
  "term_id": "GO:0003712",
  "gene_name": "Thyroid hormone receptor-associated protein 3"
}